{
  "gene": "UniProtKB:P29475",
  "gene_symbol": "NOS1",
  "term_label": "response to hormone",
  "gene_name": "Nitric oxide synthase 1",
  "term_id": "GO:0009725"
}